{
  "term_label": "neuron projection maintenance",
  "gene": "UniProtKB:Q96EK5",
  "gene_symbol": "KIFBP",
  "term_id": "GO:1990535",
  "gene_name": "KIF-binding protein"
}